protein localization to photoreceptor connecting cilium [GO:1903621] (biological process) Also known as: protein localisation in photoreceptor connecting cilium, protein localisation to photoreceptor connecting cilium, protein localization in photoreceptor connecting cilium Relationships: is a type of protein localization to non-motile cilium [GO:0097499]; is a type of protein localization to ciliary transition zone [GO:1904491] References: PMID:25398945 Sources: GOC:TermGenie, GOC:lb, GO_REF:0000087 Definition: A process in which a protein is transported to, or maintained in, a location within a photoreceptor connecting cilium.